positive regulation of glucuronoxylan catabolic process [GO:2000917] (biological process) Sources: GOC:mengo_curators Also known as: positive regulation of glucuronoxylan catabolism Subtypes: positive regulation of glucuronoarabinoxylan catabolic process [GO:2000920] Definition: Any process that activates or increases the frequency, rate or extent of glucuronoxylan catabolic process. Relationships: is a type of regulation of glucuronoxylan catabolic process [GO:2000915]; is a type of positive regulation of xylan catabolic process [GO:2001002]; positively regulates GO:2000886